alveolar lamellar body membrane [GO:0097233] (cellular component) References: PMID:11940594 Sources: GOC:sl Definition: The lipid bilayer surrounding an alveolar lamellar body, a specialized secretory organelle found in type II pneumocytes and involved in the synthesis, secretion, and reutilization of pulmonary surfactant. Relationships: is a type of lamellar body membrane [GO:0097232]; is part of alveolar lamellar body [GO:0097208]